{
  "gene": "UniProtKB:Q96KG9",
  "gene_symbol": "SCYL1",
  "gene_name": "N-terminal kinase-like protein",
  "term_label": "Unknown cellular component",
  "term_id": "UNKNOWN:0003"
}